lactose catabolic process [GO:0005990] (biological process) Sources: GOC:go_curators Relationships: is a type of lactose metabolic process [GO:0005988]; is a type of disaccharide catabolic process [GO:0046352] Also known as: lactose breakdown, lactose catabolism, lactose degradation Subtypes: lactose catabolic process via tagatose-6-phosphate [GO:0019512], lactose catabolic process, using glucoside 3-dehydrogenase [GO:0019513], lactose catabolic process via UDP-galactose [GO:0019515] Definition: The chemical reactions and pathways resulting in the breakdown of lactose, the disaccharide galactopyranosyl-glucose.